{
  "term_label": "plasma membrane",
  "gene_name": "Leukocyte immunoglobulin-like receptor subfamily A member 2",
  "term_id": "GO:0005886",
  "gene_symbol": "LILRA2",
  "gene": "UniProtKB:Q8N149"
}